intestinal phytosterol absorption [GO:0060752] (biological process) Definition: A process in which phytosterols are taken up from the contents of the intestine. Relationships: is a type of intestinal lipid absorption [GO:0098856] Regulation: negatively regulated by negative regulation of intestinal phytosterol absorption [GO:0010949] Sources: GOC:dph, GOC:tb